{
  "term_label": "endosome",
  "gene_symbol": "RAB3D",
  "term_id": "GO:0005768",
  "gene": "UniProtKB:O95716",
  "gene_name": "Ras-related protein Rab-3D"
}